{
  "gene_symbol": "MROH9",
  "gene_name": "Maestro heat-like repeat-containing protein family member 9",
  "gene": "UniProtKB:Q5TGP6",
  "term_id": "UNKNOWN:0001",
  "term_label": "Unknown molecular function"
}